{
  "gene": "UniProtKB:Q6A162",
  "term_id": "GO:0002009",
  "gene_name": "Keratin, type I cytoskeletal 40",
  "gene_symbol": "KRT40",
  "term_label": "morphogenesis of an epithelium"
}